{
  "gene": "UniProtKB:Q9BV79",
  "gene_name": "Enoyl-[acyl-carrier-protein] reductase, mitochondrial",
  "term_label": "Unknown molecular function",
  "term_id": "UNKNOWN:0001",
  "gene_symbol": "MECR"
}